4-hydroxycatechol 1,2-dioxygenase activity [GO:0047074] (molecular function) Relationships: is a type of oxidoreductase activity, acting on single donors with incorporation of molecular oxygen, incorporation of two atoms of oxygen [GO:0016702] Definition: Catalysis of the reaction: benzene-1,2,4-triol + O2 = maleylacetate + 2 H+. Sources: RHEA:35595